Golgi trans cisterna membrane [GO:1990676] (cellular component) Also known as: trans-Golgi cisterna membrane Relationships: is a type of Golgi cisterna membrane [GO:0032580]; is part of Golgi trans cisterna [GO:0000138] Definition: The lipid bilayer surrounding any of the thin, flattened compartments that form the trans portion of the Golgi complex. References: PMID:16038056, PMID:24119662 Sources: GOC:bhm